{
  "gene_name": "T cell receptor beta variable 7-8",
  "term_label": "cell surface receptor signaling pathway",
  "gene_symbol": "TRBV7-8",
  "gene": "UniProtKB:A0A1B0GX51",
  "term_id": "GO:0007166"
}